{
  "gene_symbol": "ACOX1",
  "gene": "UniProtKB:Q15067",
  "gene_name": "Peroxisomal acyl-coenzyme A oxidase 1",
  "term_id": "GO:0000038",
  "term_label": "very long-chain fatty acid metabolic process"
}